negative regulation of dopamine secretion [GO:0033602] (biological process) Definition: Any process that stops, prevents, or reduces the frequency, rate or extent of the regulated release of dopamine. Sources: GOC:sl Also known as: down regulation of dopamine secretion, down-regulation of dopamine secretion, downregulation of dopamine secretion, inhibition of dopamine secretion Relationships: is a type of regulation of dopamine secretion [GO:0014059]; is a type of negative regulation of catecholamine secretion [GO:0033604]; negatively regulates dopamine secretion [GO:0014046]